positive regulation of phosphatase activity [GO:0010922] (biological process) Definition: Any process that increases the rate or frequency of phosphatase activity. Phosphatases catalyze the hydrolysis of phosphoric monoesters, releasing inorganic phosphate. Sources: GOC:BHF, GOC:dph, GOC:tb Relationships: is a type of regulation of phosphatase activity [GO:0010921]; is_a positive regulation of dephosphorylation [GO:0035306]; is_a positive regulation of hydrolase activity [GO:0051345]; positively regulates GO:0016791 Subtypes: positive regulation of alkaline phosphatase activity [GO:0010694]